fructose-6-phosphate binding [GO:0070095] (molecular function) Definition: Binding to fructose 6-phosphate. Also known as: fructose 6-phosphate binding, D-fructose 6-phosphate binding Sources: GOC:mah Relationships: is a type of anion binding [GO:0043168]; is a type of carbohydrate derivative binding [GO:0097367]